{
  "gene_symbol": "PLEKHA8P1",
  "term_label": "cytosol",
  "gene_name": "Putative protein PLEKHA9",
  "gene": "UniProtKB:O95397",
  "term_id": "GO:0005829"
}